adenine phosphoribosyltransferase activity [GO:0003999] (MF) Definition: Catalysis of the reaction: AMP + diphosphate = adenine + 5-phospho-alpha-D-ribose 1-diphosphate. Also known as: AMP diphosphorylase activity, AMP pyrophosphorylase activity, AMP-pyrophosphate phosphoribosyltransferase activity, AMP:diphosphate phospho-D-ribosyltransferase activity, APRT activity, adenine phosphoribosylpyrophosphate transferase activity, adenosine phosphoribosyltransferase activity, adenylate pyrophosphorylase activity, adenylic pyrophosphorylase activity, transphosphoribosidase activity Relationships: is_a purine phosphoribosyltransferase activity [GO:0106130] Sources: RHEA:16609